{
  "gene_name": "ADP-ribosyl cyclase_cyclic ADP-ribose hydrolase 2",
  "term_id": "GO:0030890",
  "gene_symbol": "BST1",
  "term_label": "positive regulation of B cell proliferation",
  "gene": "UniProtKB:Q10588"
}